{
  "term_label": "CatSper complex",
  "term_id": "GO:0036128",
  "gene_symbol": "CATSPERD",
  "gene_name": "Cation channel sperm-associated auxiliary subunit delta",
  "gene": "UniProtKB:Q86XM0"
}